regulation of histamine uptake [GO:0051616] (biological process) Subtypes: GO:0051617, GO:0051618 Sources: GOC:ai Definition: Any process that modulates the frequency, rate or extent of the directed movement of the neurotransmitter histamine into a cell. Also known as: regulation of histamine import Relationships: is a type of regulation of neurotransmitter uptake [GO:0051580]; regulates histamine uptake [GO:0051615]